{
  "gene": "UniProtKB:A0A6Q8PHA8",
  "gene_name": "Uncharacterized protein",
  "term_id": "UNKNOWN:0003",
  "gene_symbol": "A0A6Q8PHA8",
  "term_label": "Unknown cellular component"
}